{
  "term_label": "Unknown molecular function",
  "gene_name": "LIX1-like protein",
  "gene": "UniProtKB:Q8IVB5",
  "term_id": "UNKNOWN:0001",
  "gene_symbol": "LIX1L"
}